{
  "term_label": "exocytosis",
  "gene": "UniProtKB:Q17RC7",
  "term_id": "GO:0006887",
  "gene_name": "Exocyst complex component 3-like protein 4",
  "gene_symbol": "EXOC3L4"
}